cinnamate reductase activity [GO:0043786] (molecular function) References: PMID:10849007 Sources: RHEA:50944 Relationships: is a type of oxidoreductase activity, acting on the CH-CH group of donors, NAD or NADP as acceptor [GO:0016628] Definition: Catalysis of the reaction: 3-phenylpropanoate + NAD+ = (E)-cinnamate + NADH + H+.